{
  "gene": "UniProtKB:Q96PP9",
  "term_label": "cellular response to type II interferon",
  "term_id": "GO:0071346",
  "gene_symbol": "GBP4",
  "gene_name": "Guanylate-binding protein 4"
}